{
  "gene": "UniProtKB:Q8WWL2",
  "gene_name": "Protein spire homolog 2",
  "term_id": "GO:0048193",
  "gene_symbol": "SPIRE2",
  "term_label": "Golgi vesicle transport"
}